{
  "term_id": "GO:0004930",
  "term_label": "G protein-coupled receptor activity",
  "gene_symbol": "GPR45",
  "gene": "UniProtKB:Q9Y5Y3",
  "gene_name": "Probable G-protein coupled receptor 45"
}